{
  "gene_name": "Putative teratocarcinoma-derived growth factor 3",
  "gene_symbol": "CRIPTO3",
  "term_label": "nodal signaling pathway",
  "term_id": "GO:0038092",
  "gene": "UniProtKB:P51864"
}